{
  "gene_name": "ATP-dependent RNA helicase A",
  "term_label": "ribonucleoprotein complex",
  "term_id": "GO:1990904",
  "gene_symbol": "DHX9",
  "gene": "UniProtKB:Q08211"
}